{
  "gene": "UniProtKB:Q9BY11",
  "term_id": "GO:1900006",
  "term_label": "positive regulation of dendrite development",
  "gene_name": "Protein kinase C and casein kinase substrate in neurons protein 1",
  "gene_symbol": "PACSIN1"
}